{
  "gene_name": "StAR-related lipid transfer protein 3",
  "gene": "UniProtKB:Q14849",
  "term_label": "vesicle tethering to endoplasmic reticulum",
  "term_id": "GO:0099044",
  "gene_symbol": "STARD3"
}